anaphase-promoting complex assembly [GO:1904824] (BP) Definition: The aggregation, arrangement and bonding together of a set of components to form an anaphase-promoting complex. References: PMID:16950791 Sources: GOC:TermGenie, GO_REF:0000079 Also known as: APC assembly, anaphase promoting complex assembly, anaphase promoting complex formation, anaphase-promoting complex formation, cyclosome assembly, cyclosome formation Relationships: is a type of protein-containing complex assembly [GO:0065003]